{
  "term_id": "GO:0005549",
  "gene": "UniProtKB:Q8NGW1",
  "term_label": "odorant binding",
  "gene_symbol": "OR6B3",
  "gene_name": "Olfactory receptor 6B3"
}